{
  "gene_name": "Protein piccolo",
  "gene": "UniProtKB:Q9Y6V0",
  "term_id": "GO:0098982",
  "gene_symbol": "PCLO",
  "term_label": "GABA-ergic synapse"
}